{
  "gene": "UniProtKB:Q9BQE4",
  "term_label": "endoplasmic reticulum unfolded protein response",
  "term_id": "GO:0030968",
  "gene_name": "Selenoprotein S",
  "gene_symbol": "SELENOS"
}